cellular response to magnesium starvation [GO:0010350] (biological process) Definition: Any process that results in a change in state or activity of a cell (in terms of movement, secretion, enzyme production, gene expression, etc.) as a result of deprivation of magnesium. Relationships: is_a cellular response to starvation [GO:0009267] References: PMID:17270009